G protein-coupled UTP receptor activity [GO:0045030] (molecular function) Relationships: is a type of GO:0071553 Definition: Combining with a nucleotide and transmitting the signal to a heterotrimeric G-protein complex to initiate a change in cell activity, activated by UTP. Sources: GOC:mah Also known as: UTP-activated nucleotide receptor activity, purinoceptor type U, uridine nucleotide receptor activity